cytoplasmic icosahedral capsid assembly [GO:0039710] (biological process) Relationships: is a type of cytoplasmic capsid assembly [GO:0039709] Definition: The assembly of an icosahedral viral capsid in the cytoplasm. Often occurs by assembling around the viral genome. Sources: VZ:1950